{
  "term_label": "Unknown biological process",
  "gene_symbol": "CYP4X1",
  "gene": "UniProtKB:Q8N118",
  "term_id": "UNKNOWN:0002",
  "gene_name": "Cytochrome P450 4X1"
}